{
  "gene": "UniProtKB:P31040",
  "gene_symbol": "SDHA",
  "term_id": "GO:0006121",
  "term_label": "mitochondrial electron transport, succinate to ubiquinone",
  "gene_name": "Succinate dehydrogenase [ubiquinone] flavoprotein subunit, mitochondrial"
}